{
  "term_id": "UNKNOWN:0002",
  "gene_name": "Transmembrane protein 229B",
  "term_label": "Unknown biological process",
  "gene_symbol": "TMEM229B",
  "gene": "UniProtKB:Q8NBD8"
}